somatostatin receptor signaling pathway [GO:0038169] (biological process) Definition: A G protein-coupled receptor signaling pathway initiated by somatostatin binding to the somatostatin receptor (SSTR) on the surface of a target cell, and ending with the regulation of a downstream cellular process. Subtypes: somatostatin signaling pathway [GO:0038170] Relationships: is a type of G protein-coupled receptor signaling pathway [GO:0007186] Also known as: SST receptor signaling pathway, SSTR signaling pathway Note: In addition to somatostatin (SST), the somatostatin receptors (SSTRs) can also be activated by the agonist cortistatin (CST). For signal transduction specifically initiated by the ligand somatostatin, consider instead annotating to the child term 'somatostatin signaling pathway ; GO:0038170'. References: PMID:18006219, PMID:8769369 Sources: GOC:jc